{
  "gene": "UniProtKB:P02686",
  "term_id": "GO:0033269",
  "term_label": "internode region of axon",
  "gene_name": "Myelin basic protein",
  "gene_symbol": "MBP"
}